{
  "term_id": "GO:0005615",
  "gene_name": "Probetacellulin",
  "term_label": "extracellular space",
  "gene": "UniProtKB:P35070",
  "gene_symbol": "BTC"
}